{
  "term_id": "GO:0070507",
  "term_label": "regulation of microtubule cytoskeleton organization",
  "gene_symbol": "TRAF3IP1",
  "gene_name": "TRAF3-interacting protein 1",
  "gene": "UniProtKB:Q8TDR0"
}